{
  "gene_name": "Probable proline--tRNA ligase, mitochondrial",
  "term_label": "prolyl-tRNA aminoacylation",
  "term_id": "GO:0006433",
  "gene": "UniProtKB:Q7L3T8",
  "gene_symbol": "PARS2"
}